{
  "gene_symbol": "DAB2",
  "gene": "UniProtKB:P98082",
  "term_id": "GO:0006898",
  "term_label": "receptor-mediated endocytosis",
  "gene_name": "Disabled homolog 2"
}